{
  "term_id": "GO:0005509",
  "gene": "UniProtKB:Q9HCY8",
  "term_label": "calcium ion binding",
  "gene_symbol": "S100A14",
  "gene_name": "Protein S100-A14"
}